{
  "gene_symbol": "PSG7",
  "term_label": "Unknown molecular function",
  "gene_name": "Pregnancy-specific beta-1-glycoprotein 7",
  "gene": "UniProtKB:Q13046",
  "term_id": "UNKNOWN:0001"
}